{
  "term_label": "Unknown cellular component",
  "term_id": "UNKNOWN:0003",
  "gene": "UniProtKB:O43280",
  "gene_name": "Trehalase",
  "gene_symbol": "TREH"
}